{
  "term_id": "GO:0005886",
  "gene_name": "Relaxin-3 receptor 1",
  "gene": "UniProtKB:Q9NSD7",
  "term_label": "plasma membrane",
  "gene_symbol": "RXFP3"
}